{
  "term_id": "UNKNOWN:0003",
  "gene": "UniProtKB:Q7L0L9",
  "term_label": "Unknown cellular component",
  "gene_name": "Transmembrane protein LOC653160",
  "gene_symbol": "Q7L0L9"
}